{
  "term_label": "microtubule associated complex",
  "gene_name": "F-box_WD repeat-containing protein 11",
  "term_id": "GO:0005875",
  "gene_symbol": "FBXW11",
  "gene": "UniProtKB:Q9UKB1"
}